{
  "term_label": "Unknown molecular function",
  "gene_name": "Non-secretory ribonuclease",
  "term_id": "UNKNOWN:0001",
  "gene": "UniProtKB:P10153",
  "gene_symbol": "RNASE2"
}